{
  "gene": "UniProtKB:P51172",
  "term_label": "plasma membrane",
  "gene_name": "Amiloride-sensitive sodium channel subunit delta",
  "term_id": "GO:0005886",
  "gene_symbol": "SCNN1D"
}